{
  "term_label": "keratin filament",
  "gene_symbol": "KRT8",
  "term_id": "GO:0045095",
  "gene": "UniProtKB:P05787",
  "gene_name": "Keratin, type II cytoskeletal 8"
}